{
  "gene": "UniProtKB:Q5W0B7",
  "term_label": "Unknown molecular function",
  "term_id": "UNKNOWN:0001",
  "gene_symbol": "TMEM236",
  "gene_name": "Transmembrane protein 236"
}